pseurotin A catabolic process [GO:1900789] (biological process) Sources: GOC:TermGenie, GOC:di Definition: The chemical reactions and pathways resulting in the breakdown of pseurotin A. Also known as: pseurotin A breakdown, pseurotin A catabolism, pseurotin A degradation, Pseurotin breakdown, Pseurotin catabolic process, Pseurotin catabolism, Pseurotin degradation Relationships: is a type of lactam catabolic process [GO:0072340]